guard cell morphogenesis [GO:0010442] (biological process) Sources: GOC:expert_db, GOC:tb Definition: Generation and organization of the polarized cell that is capable of turgor driven movement. Relationships: is a type of GO:0000902; is a type of post-embryonic plant morphogenesis [GO:0090698]; is part of guard cell development [GO:0010441] Also known as: guard cell morphogenesis during differentiation